{
  "gene_name": "Tyrosine-protein kinase Fer",
  "term_id": "GO:0006935",
  "gene": "UniProtKB:P16591",
  "gene_symbol": "FER",
  "term_label": "chemotaxis"
}